olfactory nerve maturation [GO:0021630] (biological process) Definition: A developmental process, independent of morphogenetic (shape) change, that is required for the olfactory nerve to attain its fully functional state. The olfactory nerve is a collection of sensory nerve rootlets that extend down from the olfactory bulb to the olfactory mucosa of the upper parts of the nasal cavity. This nerve conducts odor information to the brainstem. Sources: GOC:cls, GOC:dgh, GOC:dph, GOC:jid, GO_REF:0000021 Also known as: CN I maturation Relationships: is a type of cranial nerve maturation [GO:0021605]; BFO_0000050 olfactory nerve development [GO:0021553]